{
  "gene_symbol": "GPR148",
  "term_label": "membrane",
  "gene": "UniProtKB:Q8TDV2",
  "term_id": "GO:0016020",
  "gene_name": "Probable G-protein coupled receptor 148"
}